{
  "gene_name": "C-type lectin domain family 2 member B",
  "term_label": "receptor ligand activity",
  "term_id": "GO:0048018",
  "gene": "UniProtKB:Q92478",
  "gene_symbol": "CLEC2B"
}